{
  "gene_symbol": "BAIAP2",
  "term_id": "GO:0030838",
  "gene_name": "Brain-specific angiogenesis inhibitor 1-associated protein 2",
  "gene": "UniProtKB:Q9UQB8",
  "term_label": "positive regulation of actin filament polymerization"
}